{
  "term_label": "Unknown biological process",
  "gene_symbol": "KCNQ1DN",
  "gene": "UniProtKB:Q9H478",
  "gene_name": "KCNQ1 downstream neighbor protein",
  "term_id": "UNKNOWN:0002"
}